{
  "gene": "UniProtKB:Q6GPI1",
  "term_label": "serine-type endopeptidase activity",
  "gene_symbol": "CTRB2",
  "gene_name": "Chymotrypsinogen B2",
  "term_id": "GO:0004252"
}